{
  "term_id": "UNKNOWN:0003",
  "gene_name": "Rab GTPase-binding effector protein 2",
  "gene": "UniProtKB:Q9H5N1",
  "term_label": "Unknown cellular component",
  "gene_symbol": "RABEP2"
}